{
  "gene_name": "Taste receptor type 2 member 3",
  "gene": "UniProtKB:Q9NYW6",
  "term_label": "membrane",
  "gene_symbol": "TAS2R3",
  "term_id": "GO:0016020"
}